{
  "term_label": "nucleus",
  "gene": "UniProtKB:O60356",
  "gene_name": "Nuclear protein 1",
  "gene_symbol": "NUPR1",
  "term_id": "GO:0005634"
}